{
  "gene": "UniProtKB:Q86W56",
  "term_id": "GO:0006282",
  "term_label": "regulation of DNA repair",
  "gene_name": "Poly(ADP-ribose) glycohydrolase",
  "gene_symbol": "PARG"
}